regulation of membrane depolarization during action potential [GO:0098902] (biological process) Definition: Any process that modulates the rate, frequency or extent of membrane depolarization during an action potential. Membrane depolarization is the process in which membrane potential changes in the depolarizing direction from the resting potential. Relationships: is a type of GO:0003254; regulates membrane depolarization during action potential [GO:0086010] Subtypes: GO:1900825 Sources: GOC:dos, GOC:dph, GOC:tb, ISBN:978-0-07-139011-8